mesaxon [GO:0097453] (CC) Definition: Portion of the ensheathing process (either myelin or non-myelin) where the enveloping lips of the ensheathing cell come together so that their apposed plasma membranes run parallel to each other, separated by a cleft 12 nm wide. Sources: ISBN:0195065719, NIF_Subcellular:sao2127666702 Also known as: mesaxon of Schwann cell Relationships: is a type of GO:1990015